{
  "gene_symbol": "ZNF679",
  "term_id": "GO:0000978",
  "gene": "UniProtKB:Q8IYX0",
  "gene_name": "Zinc finger protein 679",
  "term_label": "RNA polymerase II cis-regulatory region sequence-specific DNA binding"
}